{
  "gene": "UniProtKB:O94778",
  "gene_name": "Aquaporin-8",
  "gene_symbol": "AQP8",
  "term_label": "water channel activity",
  "term_id": "GO:0015250"
}